{
  "gene_symbol": "GPER1",
  "term_id": "GO:0030284",
  "gene": "UniProtKB:Q99527",
  "gene_name": "G-protein coupled estrogen receptor 1",
  "term_label": "nuclear estrogen receptor activity"
}